microtubule cytoskeleton organization involved in establishment of planar polarity [GO:0090176] (biological process) Subtypes: establishment of mitotic spindle orientation involved in growth plate cartilage chondrocyte division [GO:0003425] Sources: GOC:ascb_2009, GOC:dph, GOC:tb Also known as: microtubule cytoskeleton organisation involved in establishment of planar polarity Relationships: is a type of GO:0000226; is part of establishment of planar polarity [GO:0001736] Definition: A process that is carried out at the cellular level which results in the assembly, arrangement of constituent parts, or disassembly of cytoskeletal structures comprising microtubules and their associated proteins and contributes to the establishment of planar polarity.